{
  "term_label": "GDP-mannose transmembrane transport",
  "gene_name": "Transmembrane protein 241",
  "gene": "UniProtKB:Q24JQ0",
  "term_id": "GO:1990570",
  "gene_symbol": "TMEM241"
}